negative regulation of non-motile cilium assembly [GO:1902856] (biological process) Definition: Any process that stops, prevents or reduces the frequency, rate or extent of non-motile cilium assembly. References: PMID:23807208 Sources: GOC:TermGenie, GOC:cilia, GOC:kmv, GO_REF:0000058 Also known as: inhibition of immotile primary cilium assembly, inhibition of nonmotile primary cilium assembly, inhibition of sensory cilium assembly, down regulation of immotile primary cilium assembly, down regulation of nonmotile primary cilia assembly, down regulation of nonmotile primary cilium assembly, down regulation of sensory cilium assembly, down regulation of sensory cilium biogenesis, down-regulation of immotile primary cilium assembly, down-regulation of nonmotile primary cilia assembly, down-regulation of nonmotile primary cilium assembly, down-regulation of sensory cilium assembly, down-regulation of sensory cilium biogenesis, downregulation of immotile primary cilium assembly, downregulation of nonmotile primary cilia assembly, downregulation of nonmotile primary cilium assembly, downregulation of sensory cilium assembly, downregulation of sensory cilium biogenesis, inhibition of nonmotile primary cilia assembly, inhibition of sensory cilium biogenesis, negative regulation of immotile primary cilium assembly, negative regulation of nonmotile primary cilia assembly, negative regulation of nonmotile primary cilium assembly, negative regulation of sensory cilium assembly, negative regulation of sensory cilium biogenesis Relationships: is_a negative regulation of cilium assembly [GO:1902018]; is a type of regulation of non-motile cilium assembly [GO:1902855]; negatively regulates non-motile cilium assembly [GO:1905515]